phosphatidylinositol diacylglycerol-lyase activity [GO:0004436] (molecular function) Relationships: is a type of phosphorus-oxygen lyase activity [GO:0016849] Sources: EC:4.6.1.13 Also known as: monophosphatidylinositol phosphodiesterase activity, 1-phosphatidylinositol phosphodiesterase activity, 1-phosphatidyl-1D-myo-inositol diacyl-sn-glycerol-lyase (1D-myo-inositol-1,2-cyclic-phosphate-forming), 1-phosphatidyl-1D-myo-inositol diacylglycerol-lyase (1,2-cyclic-phosphate-forming), 1-phosphatidyl-D-myo-inositol inositolphosphohydrolase (cyclic-phosphate-forming) Definition: Catalysis of the reaction: 1-phosphatidyl-1D-myo-inositol = D-myo-inositol 1,2-cyclic phosphate + diacylglycerol.